regulation of cristae formation [GO:1903850] (biological process) Note: AN example of this is PINK1 in human (Q9BXM7) in PMID:19279012 inferred from mutant phenotype Subtypes: negative regulation of cristae formation [GO:1903851], positive regulation of cristae formation [GO:1903852] Definition: Any process that modulates the frequency, rate or extent of cristae formation. Relationships: is a type of GO:0010821; regulates cristae formation [GO:0042407] References: PMID:19279012 Sources: GOC:PARL, GOC:TermGenie, GOC:pad, GO_REF:0000058